{
  "gene": "UniProtKB:P18887",
  "term_label": "Unknown molecular function",
  "gene_name": "DNA repair protein XRCC1",
  "gene_symbol": "XRCC1",
  "term_id": "UNKNOWN:0001"
}